{
  "gene_name": "DNA dC-dU-editing enzyme APOBEC-3H",
  "term_label": "cytoplasm",
  "gene": "UniProtKB:Q6NTF7",
  "term_id": "GO:0005737",
  "gene_symbol": "APOBEC3H"
}